{
  "gene": "UniProtKB:Q9HBV1",
  "term_id": "GO:0030552",
  "term_label": "cAMP binding",
  "gene_name": "Popeye domain-containing protein 3",
  "gene_symbol": "POPDC3"
}